nucleoid [GO:0009295] (cellular component) Subtypes: mitochondrial nucleoid [GO:0042645], plastid nucleoid [GO:0042646], bacterial nucleoid [GO:0043590] Definition: The region of a virus, bacterial cell, mitochondrion or chloroplast to which the nucleic acid is confined. Relationships: is a type of GO:0110165 Sources: GOC:bm, GOC:ma, ISBN:3540076689